{
  "term_label": "Unknown cellular component",
  "gene": "UniProtKB:Q8N4L8",
  "term_id": "UNKNOWN:0003",
  "gene_symbol": "CCDC24",
  "gene_name": "Coiled-coil domain-containing protein 24"
}